{
  "gene_name": "Olfactory receptor 10J1",
  "term_label": "olfactory receptor activity",
  "term_id": "GO:0004984",
  "gene_symbol": "OR10J1",
  "gene": "UniProtKB:P30954"
}